acetyl-CoA carboxylase complex [GO:0009317] (cellular component) References: PMID:12121720 Sources: GOC:jl, GOC:mah Also known as: ACCase complex Subtypes: plastid acetyl-CoA carboxylase complex [GO:0032282] Relationships: is a type of catalytic complex [GO:1902494]; is part of cytoplasm [GO:0005737] Definition: A protein complex that catalyzes the first step in long-chain fatty acid biosynthesis. For example, in E. coli the complex is heterohexameric and composed of biotin carbonyl carrier protein, biotin carboxylase and the acetate CoA-transferase complex.